regulation of systemic acquired resistance [GO:0010112] (biological process) Sources: GOC:sm Definition: Any process that modulates the frequency, rate or extent of systemic acquired resistance. Subtypes: GO:0010113, GO:1901672 Relationships: is a type of regulation of response to biotic stimulus [GO:0002831]; is a type of GO:0031347; is a type of regulation of response to external stimulus [GO:0032101]; regulates systemic acquired resistance [GO:0009627]